{
  "gene": "UniProtKB:P49788",
  "term_id": "GO:0005615",
  "term_label": "extracellular space",
  "gene_symbol": "RARRES1",
  "gene_name": "Retinoic acid receptor responder protein 1"
}